{
  "term_id": "GO:0072659",
  "gene_name": "Melanocortin-2 receptor accessory protein",
  "gene": "UniProtKB:Q8TCY5",
  "gene_symbol": "MRAP",
  "term_label": "protein localization to plasma membrane"
}